{
  "term_label": "amino acid catabolic process",
  "gene_name": "L-amino-acid oxidase",
  "gene_symbol": "IL4I1",
  "term_id": "GO:0009063",
  "gene": "UniProtKB:Q96RQ9"
}